{
  "gene_symbol": "MET",
  "gene_name": "Hepatocyte growth factor receptor",
  "gene": "UniProtKB:P08581",
  "term_label": "pancreas development",
  "term_id": "GO:0031016"
}